postsynaptic endocytosis [GO:0140239] (biological process) Definition: A vesicle-mediated transport process in which the postsynapse take up external materials or membrane constituents by the invagination of a small region of the plasma membrane to form a new membrane-bounded vesicle. References: PMID:12839988 Note: Note that this term was created for the SynGO project, and will be obsoleted when the SynGO annotations are made in Noctua. Relationships: is a type of endocytosis [GO:0006897]; is a type of establishment of localization in cell [GO:0051649]; is a type of GO:0099003; occurs in GO:0098794 Subtypes: GO:0098884